{
  "gene": "UniProtKB:Q9H0Q0",
  "gene_symbol": "CYRIA",
  "term_id": "UNKNOWN:0003",
  "term_label": "Unknown cellular component",
  "gene_name": "CYFIP-related Rac1 interactor A"
}